{
  "gene_symbol": "CFAP58",
  "term_label": "Unknown biological process",
  "gene": "UniProtKB:Q5T655",
  "term_id": "UNKNOWN:0002",
  "gene_name": "Cilia- and flagella-associated protein 58"
}